{
  "term_id": "GO:0035021",
  "gene_name": "Rho GTPase-activating protein 24",
  "term_label": "negative regulation of Rac protein signal transduction",
  "gene": "UniProtKB:Q8N264",
  "gene_symbol": "ARHGAP24"
}